{
  "gene": "UniProtKB:A8CG34",
  "gene_symbol": "POM121C",
  "term_label": "nuclear localization sequence binding",
  "gene_name": "Nuclear envelope pore membrane protein POM 121C",
  "term_id": "GO:0008139"
}